{
  "gene_name": "Putative uncharacterized protein LINC02898",
  "gene": "UniProtKB:Q6ZV80",
  "term_label": "Unknown cellular component",
  "term_id": "UNKNOWN:0003",
  "gene_symbol": "LINC02898"
}